{
  "term_id": "GO:0004722",
  "term_label": "protein serine/threonine phosphatase activity",
  "gene_symbol": "CTDNEP1",
  "gene": "UniProtKB:O95476",
  "gene_name": "CTD nuclear envelope phosphatase 1"
}